{
  "term_id": "GO:0000786",
  "gene_name": "Histone H2A type 3",
  "term_label": "nucleosome",
  "gene": "UniProtKB:Q7L7L0",
  "gene_symbol": "H2AC25"
}